regulation of single stranded viral RNA replication via double stranded DNA intermediate [GO:0045091] (biological process) Definition: Any process that modulates the frequency, rate or extent of single stranded viral RNA replication via double stranded DNA intermediate. Sources: GOC:go_curators Also known as: regulation of retroviral genome replication Relationships: is_a regulation of viral genome replication [GO:0045069]; is a type of GO:2001141; regulates single stranded viral RNA replication via double stranded DNA intermediate [GO:0039692] Subtypes: negative regulation of single stranded viral RNA replication via double stranded DNA intermediate [GO:0045869], positive regulation of single stranded viral RNA replication via double stranded DNA intermediate [GO:0045870]